poly(glucopyranosyl N-acetylgalactosamine 1-phosphate) teichoic acid biosynthetic process [GO:1902016] (biological process) Definition: The chemical reactions and pathways resulting in the formation of poly(glucopyranosyl N-acetylgalactosamine 1-phosphate) teichoic acid. Relationships: is a type of teichoic acid biosynthetic process [GO:0019350] Also known as: poly(glucopyranosyl N-acetylgalactosamine 1-phosphate) teichoic acid anabolism, poly(glucopyranosyl N-acetylgalactosamine 1-phosphate) teichoic acid biosynthesis, poly(glucopyranosyl N-acetylgalactosamine 1-phosphate) teichoic acid formation, poly(glucopyranosyl N-acetylgalactosamine 1-phosphate) teichoic acid synthesis, poly(glucosyl N-acetylgalactosamine 1-phosphate) teichoic acid biosynthesis, poly(glucosyl N-acetylgalactosamine 1-phosphate) teichoic acid biosynthetic process References: PMID:16735734 Sources: GOC:TermGenie, UniPathway:UPA00789, UniPathway:UPA00828